lens induction in camera-type eye [GO:0060235] (biological process) Relationships: is a type of developmental induction [GO:0031128]; is part of lens morphogenesis in camera-type eye [GO:0002089] Definition: Signaling at short range between the head ectoderm and the optic vesicle that results in the head ectoderm forming a lens. Sources: GOC:dph, ISBN:0878932437